{
  "gene_symbol": "CASZ1",
  "term_id": "GO:0000977",
  "term_label": "RNA polymerase II transcription regulatory region sequence-specific DNA binding",
  "gene_name": "Zinc finger protein castor homolog 1",
  "gene": "UniProtKB:Q86V15"
}